guanosine metabolic process [GO:0008617] (biological process) Definition: The chemical reactions and pathways involving guanine, guanine riboside, a nucleoside with a wide species distribution. Also known as: guanosine metabolism Relationships: is a type of purine ribonucleoside metabolic process [GO:0046128] Subtypes: GO:0046114, GO:0046115 Sources: ISBN:0198506732